{
  "term_id": "UNKNOWN:0001",
  "gene": "UniProtKB:Q6ZU65",
  "term_label": "Unknown molecular function",
  "gene_name": "Ubinuclein-2",
  "gene_symbol": "UBN2"
}